{
  "term_id": "GO:0003682",
  "term_label": "chromatin binding",
  "gene": "UniProtKB:Q9NRZ9",
  "gene_name": "Lymphoid-specific helicase",
  "gene_symbol": "HELLS"
}